limb joint morphogenesis [GO:0036022] (biological process) Sources: GOC:bf Definition: The process in which the anatomical structures of a limb joint are generated and organized. A limb joint is a flexible region that separates the rigid sections of a limb to allow movement in a controlled manner. Also known as: knee morphogenesis, leg joint morphogenesis Subtypes: embryonic skeletal limb joint morphogenesis [GO:0036023] Relationships: is a type of anatomical structure morphogenesis [GO:0009653]; is part of limb morphogenesis [GO:0035108]